{
  "gene": "UniProtKB:A0A075B6T7",
  "term_label": "Unknown molecular function",
  "gene_name": "T cell receptor alpha variable 6",
  "term_id": "UNKNOWN:0001",
  "gene_symbol": "TRAV6"
}